negative regulation of diacylglycerol biosynthetic process [GO:1900481] (biological process) Relationships: is a type of negative regulation of lipid biosynthetic process [GO:0051055]; is_a GO:1900480; negatively regulates diacylglycerol biosynthetic process [GO:0006651] Definition: Any process that stops, prevents or reduces the frequency, rate or extent of diacylglycerol biosynthetic process. Also known as: down regulation of diacylglycerol anabolism, down regulation of diacylglycerol biosynthesis, down regulation of diacylglycerol biosynthetic process, down regulation of diacylglycerol formation, down regulation of diacylglycerol synthesis, down-regulation of diacylglycerol anabolism, down-regulation of diacylglycerol biosynthesis, down-regulation of diacylglycerol biosynthetic process, down-regulation of diacylglycerol formation, down-regulation of diacylglycerol synthesis, downregulation of diacylglycerol anabolism, downregulation of diacylglycerol biosynthesis, downregulation of diacylglycerol biosynthetic process, downregulation of diacylglycerol formation, downregulation of diacylglycerol synthesis, inhibition of diacylglycerol anabolism, inhibition of diacylglycerol biosynthesis, inhibition of diacylglycerol formation, inhibition of diacylglycerol synthesis, negative regulation of diacylglycerol anabolism, negative regulation of diacylglycerol biosynthesis, negative regulation of diacylglycerol formation, negative regulation of diacylglycerol synthesis, inhibition of diacylglycerol biosynthetic process Sources: GOC:TermGenie